{
  "term_label": "Unknown molecular function",
  "term_id": "UNKNOWN:0001",
  "gene_symbol": "Q1T7F1",
  "gene_name": "Putative chemokine-related protein B42",
  "gene": "UniProtKB:Q1T7F1"
}